regulation of macrophage proliferation [GO:0120040] (biological process) Subtypes: positive regulation of macrophage proliferation [GO:0120041], negative regulation of macrophage proliferation [GO:0120042] Sources: GOC:BHF, GOC:BHF_miRNA, GOC:rph Definition: Any process that modulates the frequency, rate or extent of macrophage proliferation. Relationships: is a type of regulation of leukocyte proliferation [GO:0070663]; regulates macrophage proliferation [GO:0061517]